cerebellum maturation [GO:0021590] (BP) Sources: GOC:cls, GOC:dgh, GOC:dph, GOC:jid, GO_REF:0000021 Relationships: is a type of anatomical structure maturation [GO:0071695]; is part of GO:0021549; is part of hindbrain maturation [GO:0021578] Definition: A developmental process, independent of morphogenetic (shape) change, that is required for the cerebellum to attain its fully functional state. The cerebellum is the portion of the brain in the back of the head between the cerebrum and the pons. The cerebellum controls balance for walking and standing, modulates the force and range of movement and is involved in the learning of motor skills.